{
  "gene_name": "Protein KRI1 homolog",
  "term_label": "nucleolus",
  "gene": "UniProtKB:Q8N9T8",
  "term_id": "GO:0005730",
  "gene_symbol": "KRI1"
}